blood vessel lumen ensheathment [GO:0097496] (biological process) Definition: A blood vessel lumenization process that occurs by blood vessel endothelial cells delaminating and aligning along the inner surface of an existing luminal space, extending the open ended lumen, and joining to other blood vessels to form a complete blood vessel. References: PMID:23698350 Sources: GOC:dgh Relationships: is a type of blood vessel lumenization [GO:0072554]